{
  "term_id": "GO:0008453",
  "gene_name": "Alanine--glyoxylate aminotransferase",
  "term_label": "alanine-glyoxylate transaminase activity",
  "gene": "UniProtKB:P21549",
  "gene_symbol": "AGXT"
}